{
  "gene": "UniProtKB:O95813",
  "term_label": "determination of heart left/right asymmetry",
  "term_id": "GO:0061371",
  "gene_name": "Cerberus",
  "gene_symbol": "CER1"
}